positive regulation of Schwann cell migration [GO:1900149] (biological process) Definition: Any process that activates or increases the frequency, rate or extent of Schwann cell migration. Subtypes: GO:1904268 Relationships: is a type of regulation of Schwann cell migration [GO:1900147]; is a type of positive regulation of glial cell migration [GO:1903977]; positively regulates Schwann cell migration [GO:0036135] Sources: GOC:TermGenie, GOC:sjw Also known as: up regulation of Schwann cell migration, up-regulation of Schwann cell migration, upregulation of Schwann cell migration, activation of Schwann cell migration